{
  "gene_symbol": "PGLYRP4",
  "term_label": "immune response",
  "term_id": "GO:0006955",
  "gene": "UniProtKB:Q96LB8",
  "gene_name": "Peptidoglycan recognition protein 4"
}